{
  "gene": "UniProtKB:Q8IV32",
  "gene_symbol": "CCDC71",
  "term_id": "UNKNOWN:0003",
  "gene_name": "Coiled-coil domain-containing protein 71",
  "term_label": "Unknown cellular component"
}